{
  "gene_symbol": "FOXR2",
  "gene_name": "Forkhead box protein R2",
  "term_id": "GO:1990837",
  "term_label": "sequence-specific double-stranded DNA binding",
  "gene": "UniProtKB:Q6PJQ5"
}